{
  "gene_name": "Cation channel sperm-associated auxiliary subunit beta",
  "term_label": "Unknown molecular function",
  "gene": "UniProtKB:Q9H7T0",
  "term_id": "UNKNOWN:0001",
  "gene_symbol": "CATSPERB"
}